{
  "gene_symbol": "TUBA4B",
  "gene_name": "Putative tubulin-like protein alpha-4B",
  "gene": "UniProtKB:Q9H853",
  "term_label": "Unknown molecular function",
  "term_id": "UNKNOWN:0001"
}